{
  "gene_symbol": "KAT5",
  "gene_name": "Histone acetyltransferase KAT5",
  "term_id": "GO:0046972",
  "gene": "UniProtKB:Q92993",
  "term_label": "histone H4K16 acetyltransferase activity"
}